{
  "gene_name": "Polyglutamylase complex subunit TTLL1",
  "term_id": "GO:0007288",
  "term_label": "sperm axoneme assembly",
  "gene": "UniProtKB:O95922",
  "gene_symbol": "TTLL1"
}